paromomycin catabolic process [GO:1901154] (biological process) Sources: GOC:TermGenie, GOC:yaf, UniPathway:UPA00970 Definition: The chemical reactions and pathways resulting in the breakdown of paromomycin. Also known as: paromomycin breakdown, paromomycin catabolism, paromomycin degradation Relationships: is a type of GO:0030649; is a type of polyol catabolic process [GO:0046174]